{
  "term_label": "membrane",
  "term_id": "GO:0016020",
  "gene_symbol": "KCNV2",
  "gene": "UniProtKB:Q8TDN2",
  "gene_name": "Potassium voltage-gated channel subfamily V member 2"
}